{
  "gene": "UniProtKB:Q9H0Y0",
  "gene_symbol": "ATG10",
  "gene_name": "Ubiquitin-like-conjugating enzyme ATG10",
  "term_label": "Atg12 conjugating enzyme activity",
  "term_id": "GO:0061651"
}